{
  "term_label": "extrinsic apoptotic signaling pathway in absence of ligand",
  "term_id": "GO:0097192",
  "gene_symbol": "CASP2",
  "gene_name": "Caspase-2",
  "gene": "UniProtKB:P42575"
}